{
  "term_label": "mismatch repair",
  "term_id": "GO:0006298",
  "gene_name": "Exonuclease 1",
  "gene_symbol": "EXO1",
  "gene": "UniProtKB:Q9UQ84"
}